{
  "gene_name": "Sodium-coupled neutral amino acid transporter 5",
  "gene_symbol": "SLC38A5",
  "term_label": "glutamine transport",
  "gene": "UniProtKB:Q8WUX1",
  "term_id": "GO:0006868"
}